{
  "gene_symbol": "DLG3",
  "gene_name": "Disks large homolog 3",
  "term_id": "GO:0035418",
  "gene": "UniProtKB:Q92796",
  "term_label": "protein localization to synapse"
}